{
  "term_label": "signaling receptor binding",
  "term_id": "GO:0005102",
  "gene": "UniProtKB:Q6ZUJ8",
  "gene_name": "Phosphoinositide 3-kinase adapter protein 1",
  "gene_symbol": "PIK3AP1"
}